{
  "term_label": "plasma membrane",
  "gene_name": "ATP-sensitive inward rectifier potassium channel 8",
  "term_id": "GO:0005886",
  "gene_symbol": "KCNJ8",
  "gene": "UniProtKB:Q15842"
}